{
  "term_label": "host-mediated suppression of symbiont invasion",
  "gene_name": "Interferon-induced transmembrane protein 3",
  "gene": "UniProtKB:Q01628",
  "gene_symbol": "IFITM3",
  "term_id": "GO:0046597"
}